glucosinolate catabolic process [GO:0019762] (biological process) Sources: GOC:ai Definition: The chemical reactions and pathways resulting in the breakdown of glucosinolates, substituted thioglucosides found in rapeseed products and related cruciferae. Relationships: is a type of S-glycoside catabolic process [GO:0016145]; is a type of glucosinolate metabolic process [GO:0019760] Subtypes: indole glucosinolate catabolic process [GO:0042344] Also known as: glucosinolate breakdown, glucosinolate catabolism, glucosinolate degradation